pentose-phosphate shunt, oxidative branch [GO:0009051] (biological process) Definition: The branch of the pentose-phosphate shunt which involves the oxidation of glucose 6-P and produces ribulose 5-P, reduced NADP+ and carbon dioxide (CO2). Also known as: oxidative branch, pentose pathway, oxidative pentose phosphate pathway, pentose phosphate pathway, oxidative branch, pentose phosphate shunt, oxidative branch, pentose-phosphate pathway, oxidative branch Sources: ISBN:0198506732, MetaCyc:OXIDATIVEPENT-PWY Relationships: is a type of NADPH regeneration [GO:0006740]; is a type of carbohydrate derivative metabolic process [GO:1901135]; BFO_0000050 pentose-phosphate shunt [GO:0006098]; has part glucose-6-phosphate dehydrogenase activity [GO:0004345]; has part phosphogluconate dehydrogenase (decarboxylating) activity [GO:0004616]; has part GO:0017057